{
  "gene_symbol": "OR2AK2",
  "gene_name": "Olfactory receptor 2AK2",
  "gene": "UniProtKB:Q8NG84",
  "term_id": "GO:0050911",
  "term_label": "detection of chemical stimulus involved in sensory perception of smell"
}